{
  "term_label": "intracellular glucose homeostasis",
  "term_id": "GO:0001678",
  "gene": "UniProtKB:P19367",
  "gene_name": "Hexokinase-1",
  "gene_symbol": "HK1"
}